{
  "term_id": "GO:0001228",
  "gene_name": "Transcription factor SOX-7",
  "term_label": "DNA-binding transcription activator activity, RNA polymerase II-specific",
  "gene_symbol": "SOX7",
  "gene": "UniProtKB:Q9BT81"
}